{
  "gene": "UniProtKB:Q96RD7",
  "gene_symbol": "PANX1",
  "term_label": "wide pore channel activity",
  "term_id": "GO:0022829",
  "gene_name": "Pannexin-1"
}